{
  "gene_symbol": "TRAV20",
  "term_label": "Unknown cellular component",
  "gene_name": "T cell receptor alpha variable 20",
  "term_id": "UNKNOWN:0003",
  "gene": "UniProtKB:A0A0B4J274"
}